{
  "gene_name": "Ubiquinol-cytochrome-c reductase complex assembly factor 6",
  "term_label": "mitochondrion",
  "term_id": "GO:0005739",
  "gene": "UniProtKB:Q69YU5",
  "gene_symbol": "UQCC6"
}